{
  "gene_symbol": "CYB5R1",
  "gene_name": "NADH-cytochrome b5 reductase 1",
  "term_id": "UNKNOWN:0002",
  "gene": "UniProtKB:Q9UHQ9",
  "term_label": "Unknown biological process"
}